{
  "term_label": "regulation of dendrite morphogenesis",
  "term_id": "GO:0048814",
  "gene": "UniProtKB:Q9Y250",
  "gene_symbol": "LZTS1",
  "gene_name": "Leucine zipper putative tumor suppressor 1"
}